positive regulation of hepatocyte proliferation [GO:2000347] (biological process) Sources: GOC:BHF, GOC:mah Relationships: is a type of positive regulation of epithelial cell proliferation [GO:0050679]; is a type of regulation of hepatocyte proliferation [GO:2000345]; positively regulates hepatocyte proliferation [GO:0072574] Definition: Any process that activates or increases the frequency, rate or extent of hepatocyte proliferation.